{
  "term_label": "microtubule binding",
  "term_id": "GO:0008017",
  "gene": "UniProtKB:P50570",
  "gene_name": "Dynamin-2",
  "gene_symbol": "DNM2"
}